pole cell fate determination [GO:0007278] (biological process) Relationships: is a type of cell fate determination [GO:0001709]; is a type of developmental process involved in reproduction [GO:0003006]; is part of pole cell development [GO:0007277] Sources: GOC:go_curators Definition: The cell fate determination process in which a cell becomes capable of differentiating autonomously into a pole cell regardless of its environment; upon determination, the cell fate cannot be reversed.